{
  "term_label": "Unknown cellular component",
  "gene": "UniProtKB:Q6P0A1",
  "gene_name": "Protein FAM180B",
  "term_id": "UNKNOWN:0003",
  "gene_symbol": "FAM180B"
}